{
  "gene_name": "Nucleus accumbens-associated protein 2",
  "gene": "UniProtKB:Q96BF6",
  "term_label": "DNA-binding transcription factor activity, RNA polymerase II-specific",
  "gene_symbol": "NACC2",
  "term_id": "GO:0000981"
}